{
  "term_id": "GO:0000977",
  "gene_name": "Factor in the germline alpha",
  "gene": "UniProtKB:Q6QHK4",
  "term_label": "RNA polymerase II transcription regulatory region sequence-specific DNA binding",
  "gene_symbol": "FIGLA"
}